{
  "gene_name": "Cytochrome c oxidase subunit 6A2, mitochondrial",
  "term_label": "mitochondrial electron transport, cytochrome c to oxygen",
  "term_id": "GO:0006123",
  "gene": "UniProtKB:Q02221",
  "gene_symbol": "COX6A2"
}